mitochondrial inner boundary membrane [GO:0097002] (cellular component) Also known as: inner bounding mitochondrial membrane References: PMID:16054341, PMID:19019989 Sources: GOC:mcc Relationships: is a type of cellular anatomical structure [GO:0110165]; is part of GO:0005743 Definition: The portion of the mitochondrial inner membrane that is not invaginated to form cristae. The inner boundary membrane lies parallel to the outer membrane.